protein asparagine deamidase activity [GO:0160260] (molecular function) Definition: Catalysis of the reaction: L-asparaginyl-[protein] + H2O = L-aspartyl-[protein] + NH4+. References: PMID:25752576, PMID:30092200, PMID:39719712, PMID:40240600 Sources: RHEA:57416 Relationships: is a type of GO:0016811; is a type of GO:0140096 Subtypes: protein-N-terminal asparagine amidohydrolase activity [GO:0008418], GO:0160261